positive regulation of D-aspartate import across plasma membrane [GO:0140217] (biological process) Definition: Any process that activates or increases the frequency, rate or extent of the directed import of D-aspartate from the extracellular region across the plasma membrane and into the cytosol. Relationships: is a type of positive regulation of organic acid transport [GO:0032892]; is a type of positive regulation of transmembrane transport [GO:0034764]; is a type of GO:0051957; is a type of GO:0140215; positively regulates D-aspartate import across plasma membrane [GO:0070779] References: PMID:27663541